generative cell nucleus [GO:0048555] (cellular component) Sources: GOC:tair_curators Definition: The nucleus of the generative cell, a cell contained within the pollen grain that will divide to produce two haploid sperm cells. Relationships: is a type of nucleus [GO:0005634] Also known as: male germ cell nucleus, sperm cell nucleus